{
  "term_label": "Unknown molecular function",
  "term_id": "UNKNOWN:0001",
  "gene_name": "MORN repeat-containing protein 4",
  "gene_symbol": "MORN4",
  "gene": "UniProtKB:Q8NDC4"
}